peptide stabilization [GO:0050822] (biological process) Sources: GOC:ai Also known as: peptide stabilisation, peptide stabilization activity Relationships: is a type of GO:0006518 Definition: Any process involved in maintaining the structure and integrity of a peptide and preventing it from being degraded. Subtypes: GO:0050823